{
  "gene_name": "Urotensin-2",
  "term_label": "regulation of blood pressure",
  "gene": "UniProtKB:O95399",
  "term_id": "GO:0008217",
  "gene_symbol": "UTS2"
}